negative regulation of membrane depolarization [GO:1904180] (BP) Also known as: down regulation of membrane depolarization, down-regulation of membrane depolarization, downregulation of membrane depolarization, inhibition of membrane depolarization Subtypes: negative regulation of mitochondrial depolarization [GO:0051902], negative regulation of membrane depolarization during cardiac muscle cell action potential [GO:1900826], GO:1904198 Definition: Any process that stops, prevents or reduces the frequency, rate or extent of membrane depolarization. Relationships: is a type of GO:0003254; is a type of negative regulation of biological process [GO:0048519]; negatively regulates GO:0051899 References: PMID:20826763 Sources: GOC:TermGenie, GO_REF:0000058